{
  "gene_symbol": "ICAM1",
  "gene_name": "Intercellular adhesion molecule 1",
  "term_label": "integrin binding",
  "gene": "UniProtKB:P05362",
  "term_id": "GO:0005178"
}